{
  "gene": "UniProtKB:Q9P2K6",
  "gene_symbol": "KLHL42",
  "gene_name": "Kelch-like protein 42",
  "term_id": "GO:0043161",
  "term_label": "proteasome-mediated ubiquitin-dependent protein catabolic process"
}